K48-linked deubiquitinase activity [GO:1990380] (molecular function) Definition: Hydrolysis of a ubiquitin unit from a ubiquitinated protein linked via the Lys48 residue of ubiquitin. References: PMID:22970133 Sources: GOC:PARL, GOC:bf Also known as: K48-specific deubiquitinase activity, K48-specific deubiquitinating activity, Lys48-specific deubiquitinase activity Relationships: is a type of deubiquitinase activity [GO:0101005]